{
  "gene_name": "Zinc finger protein 639",
  "gene": "UniProtKB:Q9UID6",
  "term_id": "GO:0006357",
  "term_label": "regulation of transcription by RNA polymerase II",
  "gene_symbol": "ZNF639"
}